{
  "term_label": "retromer complex binding",
  "term_id": "GO:1905394",
  "gene_name": "CapZ-interacting protein",
  "gene_symbol": "RCSD1",
  "gene": "UniProtKB:Q6JBY9"
}